{
  "gene_name": "Proline-rich transmembrane protein 1",
  "term_label": "postsynaptic membrane",
  "gene": "UniProtKB:Q99946",
  "term_id": "GO:0045211",
  "gene_symbol": "PRRT1"
}